{
  "term_label": "phosphatidylinositol-4,5-bisphosphate binding",
  "gene_symbol": "AMER1",
  "gene": "UniProtKB:Q5JTC6",
  "gene_name": "APC membrane recruitment protein 1",
  "term_id": "GO:0005546"
}